{
  "gene_symbol": "CNTNAP1",
  "term_id": "GO:0045202",
  "term_label": "synapse",
  "gene": "UniProtKB:P78357",
  "gene_name": "Contactin-associated protein 1"
}